{
  "gene_name": "DNA-directed primase_polymerase protein",
  "term_label": "mitochondrial matrix",
  "term_id": "GO:0005759",
  "gene": "UniProtKB:Q96LW4",
  "gene_symbol": "PRIMPOL"
}